maintenance of protein localization in endoplasmic reticulum [GO:0035437] (biological process) Definition: Any process in which a protein is maintained in the endoplasmic reticulum and prevented from moving elsewhere. These include sequestration within the endoplasmic reticulum, protein stabilization to prevent transport elsewhere and the active retrieval of proteins that escape the endoplasmic reticulum. Relationships: is a type of maintenance of protein localization in organelle [GO:0072595]; is part of protein localization to endoplasmic reticulum [GO:0070972]; occurs in endoplasmic reticulum [GO:0005783] Subtypes: protein retention in ER lumen [GO:0006621], SREBP-SCAP complex retention in endoplasmic reticulum [GO:0036316] Sources: GOC:bf, GOC:vw Also known as: maintenance of protein localisation in endoplasmic reticulum, maintenance of protein localization in ER, maintenance of protein location in ER, maintenance of protein location in endoplasmic reticulum, protein-ER retention, protein-endoplasmic reticulum retention, retention of protein in ER, retention of protein in endoplasmic reticulum